{
  "gene_symbol": "LIN54",
  "gene": "UniProtKB:Q6MZP7",
  "term_id": "GO:0005634",
  "term_label": "nucleus",
  "gene_name": "Protein lin-54 homolog"
}